inositol hexakisphosphate 5-phosphatase activity [GO:0050533] (molecular function) Also known as: 5-phytase activity, myo-inositol-hexakisphosphate 5-phosphohydrolase activity Sources: RHEA:13001 Relationships: is a type of inositol hexakisphosphate phosphatase activity [GO:0004446] Definition: Catalysis of the reaction: 1D-myo-inositol hexakisphosphate + H2O = 1D-myo-inositol 1,2,3,4,6-pentakisphosphate + phosphate.